{
  "gene_name": "Transient receptor potential cation channel subfamily V member 2",
  "term_label": "calcium channel activity",
  "gene_symbol": "TRPV2",
  "gene": "UniProtKB:Q9Y5S1",
  "term_id": "GO:0005262"
}